{
  "gene_name": "Probable E3 ubiquitin-protein ligase MARCHF10",
  "term_id": "UNKNOWN:0002",
  "term_label": "Unknown biological process",
  "gene": "UniProtKB:Q8NA82",
  "gene_symbol": "MARCHF10"
}